{
  "term_id": "UNKNOWN:0002",
  "gene_symbol": "LOC84773-CYHR1",
  "term_label": "Unknown biological process",
  "gene": "UniProtKB:E9PQ42",
  "gene_name": "TRAF-type domain-containing protein (Fragment)"
}